cyanide catabolic process [GO:0019500] (biological process) Also known as: cyanide breakdown, cyanide catabolism, cyanide degradation Relationships: is a type of catabolic process [GO:0009056]; is a type of cyanide metabolic process [GO:0019499] Definition: The chemical reactions and pathways resulting in the breakdown of cyanide, NC-, the anion of hydrocyanic acid. Cyanide is a potent inhibitor of respiration. Sources: ISBN:0198506732